{
  "term_id": "UNKNOWN:0001",
  "gene_name": "Transmembrane protein 132E",
  "gene_symbol": "TMEM132E",
  "gene": "UniProtKB:Q6IEE7",
  "term_label": "Unknown molecular function"
}